muscle hypertrophy in response to stress [GO:0003299] (BP) Definition: The enlargement or overgrowth of all or part of a muscle organ or tissue due to an increase in the size of its muscle cells as a result of a disturbance in organismal or cellular homeostasis. Sources: GOC:mtg_heart Relationships: is a type of response to stress [GO:0006950]; is_a muscle hypertrophy [GO:0014896]; is a type of muscle adaptation [GO:0043500] Subtypes: cardiac muscle hypertrophy in response to stress [GO:0014898]